{
  "gene_symbol": "SEPTIN3",
  "gene_name": "Neuronal-specific septin-3",
  "term_label": "septin ring",
  "term_id": "GO:0005940",
  "gene": "UniProtKB:Q9UH03"
}